{
  "gene_name": "Popeye domain-containing protein 2",
  "term_label": "striated muscle cell differentiation",
  "term_id": "GO:0051146",
  "gene": "UniProtKB:Q9HBU9",
  "gene_symbol": "POPDC2"
}